{
  "gene": "UniProtKB:Q8N6T7",
  "term_id": "GO:0000122",
  "term_label": "negative regulation of transcription by RNA polymerase II",
  "gene_symbol": "SIRT6",
  "gene_name": "NAD-dependent protein deacylase sirtuin-6"
}